{
  "gene_name": "Vasoactive intestinal polypeptide receptor 1",
  "gene": "UniProtKB:P32241",
  "term_label": "vasoactive intestinal polypeptide receptor activity",
  "gene_symbol": "VIPR1",
  "term_id": "GO:0004999"
}